{
  "term_id": "GO:0000175",
  "gene": "UniProtKB:Q9BQ65",
  "term_label": "3'-5'-RNA exonuclease activity",
  "gene_symbol": "USB1",
  "gene_name": "U6 snRNA phosphodiesterase 1"
}